{
  "term_id": "GO:0030488",
  "gene": "UniProtKB:Q9UET6",
  "gene_symbol": "FTSJ1",
  "term_label": "tRNA methylation",
  "gene_name": "Putative tRNA (cytidine(32)_guanosine(34)-2'-O)-methyltransferase"
}